{
  "gene_name": "T cell receptor alpha joining 18 (Fragment)",
  "term_label": "Unknown molecular function",
  "term_id": "UNKNOWN:0001",
  "gene": "UniProtKB:A0A075B6X9",
  "gene_symbol": "TRAJ18"
}